{
  "gene_symbol": "STRCP1",
  "term_label": "cell-matrix adhesion",
  "gene": "UniProtKB:A6NGW2",
  "term_id": "GO:0007160",
  "gene_name": "Putative stereocilin-like protein"
}